{
  "gene": "UniProtKB:Q96LY2",
  "gene_symbol": "CCDC74B",
  "gene_name": "Coiled-coil domain-containing protein 74B",
  "term_label": "Unknown biological process",
  "term_id": "UNKNOWN:0002"
}